{
  "gene_name": "Transmembrane protein 11, mitochondrial",
  "gene": "UniProtKB:P17152",
  "term_label": "mitochondrial inner membrane",
  "gene_symbol": "TMEM11",
  "term_id": "GO:0005743"
}